{
  "gene": "UniProtKB:Q12950",
  "gene_name": "Forkhead box protein D4",
  "gene_symbol": "FOXD4",
  "term_id": "GO:0009653",
  "term_label": "anatomical structure morphogenesis"
}